terpene metabolic process [GO:0042214] (BP) Definition: The chemical reactions and pathways involving terpenes, any of a large group of hydrocarbons that are made up of isoprene (C5H8) units which may be cyclic, acyclic or multicyclic, saturated or unsaturated, and may contain various functional groups. Sources: GOC:curators Also known as: terpene metabolism Relationships: is a type of GO:0006720; is_a hydrocarbon metabolic process [GO:0120252] Subtypes: carotene metabolic process [GO:0016119], GO:0033331, isoprene metabolic process [GO:0043611], GO:0043692, GO:0046246, terpene catabolic process [GO:0046247], GO:0051761